{
  "term_id": "GO:0004298",
  "gene_symbol": "TASP1",
  "gene": "UniProtKB:Q9H6P5",
  "gene_name": "Threonine aspartase 1",
  "term_label": "threonine-type endopeptidase activity"
}